{
  "term_label": "Unknown molecular function",
  "gene": "UniProtKB:Q96DI7",
  "gene_symbol": "SNRNP40",
  "gene_name": "U5 small nuclear ribonucleoprotein 40 kDa protein",
  "term_id": "UNKNOWN:0001"
}